{
  "term_id": "GO:0031507",
  "gene_name": "SWI_SNF-related matrix-associated actin-dependent regulator of chromatin subfamily A member 5",
  "gene": "UniProtKB:O60264",
  "term_label": "heterochromatin formation",
  "gene_symbol": "SMARCA5"
}